{
  "term_label": "JNK cascade",
  "gene_symbol": "MAP3K15",
  "gene": "UniProtKB:Q6ZN16",
  "gene_name": "Mitogen-activated protein kinase kinase kinase 15",
  "term_id": "GO:0007254"
}